{
  "term_label": "Unknown molecular function",
  "gene_symbol": "MAGEE1",
  "term_id": "UNKNOWN:0001",
  "gene_name": "Melanoma-associated antigen E1",
  "gene": "UniProtKB:Q9HCI5"
}